{
  "term_label": "RNA polymerase I complex",
  "gene_symbol": "POLR1A",
  "gene_name": "DNA-directed RNA polymerase I subunit RPA1",
  "term_id": "GO:0005736",
  "gene": "UniProtKB:O95602"
}